{
  "gene": "UniProtKB:Q96A49",
  "gene_name": "Synapse-associated protein 1",
  "term_label": "cytoplasm",
  "gene_symbol": "SYAP1",
  "term_id": "GO:0005737"
}